{
  "gene_symbol": "CRABP1",
  "term_id": "GO:0015908",
  "gene": "UniProtKB:P29762",
  "term_label": "fatty acid transport",
  "gene_name": "Cellular retinoic acid-binding protein 1"
}